{
  "gene_symbol": "HAAO",
  "term_label": "'de novo' NAD+ biosynthetic process from L-tryptophan",
  "gene": "UniProtKB:P46952",
  "gene_name": "3-hydroxyanthranilate 3,4-dioxygenase",
  "term_id": "GO:0034354"
}